{
  "gene_name": "AarF domain-containing protein kinase 1",
  "term_label": "Unknown molecular function",
  "gene_symbol": "ADCK1",
  "term_id": "UNKNOWN:0001",
  "gene": "UniProtKB:Q86TW2"
}